lauric acid metabolic process [GO:0048252] (biological process) Definition: The chemical reactions and pathways involving lauric acid, a fatty acid with the formula CH3(CH2)10COOH. Derived from vegetable sources. References: PMID:15555597 Sources: GOC:jid Also known as: lauric acid metabolism, n-dodecanoic acid metabolic process, n-dodecanoic acid metabolism Relationships: is a type of medium-chain fatty acid metabolic process [GO:0051791]